{
  "gene": "UniProtKB:Q6PIF2",
  "term_label": "Unknown biological process",
  "gene_name": "Synaptonemal complex central element protein 2",
  "gene_symbol": "SYCE2",
  "term_id": "UNKNOWN:0002"
}